{
  "gene_name": "Outer mitochondrial transmembrane helix translocase",
  "term_id": "GO:0140570",
  "term_label": "extraction of mislocalized protein from mitochondrial outer membrane",
  "gene": "UniProtKB:Q8NBU5",
  "gene_symbol": "ATAD1"
}